{
  "gene_name": "Alanine aminotransferase 1",
  "term_label": "Unknown cellular component",
  "gene": "UniProtKB:P24298",
  "term_id": "UNKNOWN:0003",
  "gene_symbol": "GPT"
}